epoxygenase P450 pathway [GO:0019373] (biological process) References: PMID:17979511 Sources: GOC:mah Relationships: is a type of arachidonate metabolic process [GO:0019369] Definition: The chemical reactions and pathways by which arachidonic acid is converted to other compounds including epoxyeicosatrienoic acids and dihydroxyeicosatrienoic acids.